{
  "term_label": "regulation of neurogenesis",
  "gene_name": "Hairy_enhancer-of-split related with YRPW motif protein 2",
  "gene": "UniProtKB:Q9UBP5",
  "term_id": "GO:0050767",
  "gene_symbol": "HEY2"
}